{
  "gene_name": "Complement C1q tumor necrosis factor-related protein 8",
  "term_id": "UNKNOWN:0002",
  "term_label": "Unknown biological process",
  "gene": "UniProtKB:P60827",
  "gene_symbol": "C1QTNF8"
}